{
  "term_label": "Unknown biological process",
  "term_id": "UNKNOWN:0002",
  "gene": "UniProtKB:P21926",
  "gene_symbol": "CD9",
  "gene_name": "CD9 antigen"
}